regulation of G1/S transition of mitotic cell cycle [GO:2000045] (biological process) Note: Note that this process is usually achieved by the regulation of the G1 cyclin-dependent protein kinase, consider annotating to the child term 'regulation of cyclin-dependent protein kinase activity involved in G1/S ; GO:0031657'. Subtypes: positive regulation of G1/S transition of mitotic cell cycle [GO:1900087], negative regulation of G1/S transition of mitotic cell cycle [GO:2000134] Definition: Any signaling pathway that modulates the activity of a cell cycle cyclin-dependent protein kinase to modulate the switch from G1 phase to S phase of the mitotic cell cycle. Sources: GOC:mtg_cell_cycle Relationships: is a type of regulation of mitotic cell cycle phase transition [GO:1901990]; is a type of regulation of cell cycle G1/S phase transition [GO:1902806]; regulates GO:0000082